{
  "term_id": "GO:0042789",
  "gene_symbol": "POLR2A",
  "gene": "UniProtKB:P24928",
  "term_label": "mRNA transcription by RNA polymerase II",
  "gene_name": "DNA-directed RNA polymerase II subunit RPB1"
}